sperm flagellum assembly [GO:0120316] (biological process) Definition: The assembly and organization of the sperm flagellum, the microtubule-based axoneme and associated structures that are part of a sperm flagellum (or cilium). Relationships: is a type of developmental process involved in reproduction [GO:0003006]; is a type of motile cilium assembly [GO:0044458]; is part of spermatid development [GO:0007286]; is part of GO:0030317 References: PMID:32791035 Sources: GOC:krc